{
  "gene_name": "LanC-like protein 2",
  "term_id": "GO:0009787",
  "term_label": "regulation of abscisic acid-activated signaling pathway",
  "gene": "UniProtKB:Q9NS86",
  "gene_symbol": "LANCL2"
}